{
  "gene_name": "Actin-like protein 6A",
  "term_id": "GO:0007399",
  "gene_symbol": "ACTL6A",
  "gene": "UniProtKB:O96019",
  "term_label": "nervous system development"
}